female germline ring canal stabilization [GO:0008335] (biological process) Relationships: is a type of actomyosin structure organization [GO:0031032]; is part of ovarian nurse cell to oocyte transport [GO:0007300] Definition: Maintenance of the structural integrity of the ring canals connecting the female germline cyst. Sources: GOC:curators Also known as: nurse cell ring canal stabilization, ovarian ring canal stabilization